{
  "term_id": "UNKNOWN:0002",
  "term_label": "Unknown biological process",
  "gene_name": "Protein ATP6V1FNB",
  "gene": "UniProtKB:A0A1B0GUX0",
  "gene_symbol": "ATP6V1FNB"
}